cellular response to heat [GO:0034605] (biological process) Relationships: is a type of response to heat [GO:0009408]; is a type of GO:0033554 Regulation: RO_0002211 by regulation of cellular response to heat [GO:1900034]; negatively regulated by negative regulation of cellular response to heat [GO:1900035]; positively regulated by positive regulation of cellular response to heat [GO:1900036] Definition: Any process that results in a change in state or activity of a cell (in terms of movement, secretion, enzyme production, gene expression, etc.) as a result of a heat stimulus, a temperature stimulus above the optimal temperature for that organism. Subtypes: mRNA export from nucleus in response to heat stress [GO:0031990], heat shock-mediated polytene chromosome puffing [GO:0035080], cellular heat acclimation [GO:0070370] Also known as: cellular response to heat stress Sources: GOC:mah